{
  "term_label": "early endosome",
  "gene": "UniProtKB:A8K0Z3",
  "gene_symbol": "WASHC1",
  "term_id": "GO:0005769",
  "gene_name": "WASH complex subunit 1"
}